{
  "term_id": "GO:0005829",
  "term_label": "cytosol",
  "gene_name": "Glucose-induced degradation protein 8 homolog",
  "gene": "UniProtKB:Q9NWU2",
  "gene_symbol": "GID8"
}